positive regulation of protein monoubiquitination [GO:1902527] (biological process) Note: An example is BIRC2 (UniProt ID Q13490) in PMID:21931591. Relationships: is a type of positive regulation of protein ubiquitination [GO:0031398]; is a type of GO:1902525; positively regulates protein monoubiquitination [GO:0006513] References: PMID:21931591 Sources: GOC:TermGenie Also known as: positive regulation of protein monoubiquitinylation, positive regulation of protein monoubiquitylation, up regulation of protein monoubiquitination, up regulation of protein monoubiquitinylation, up regulation of protein monoubiquitylation, up-regulation of protein monoubiquitination, up-regulation of protein monoubiquitinylation, up-regulation of protein monoubiquitylation, upregulation of protein monoubiquitination, upregulation of protein monoubiquitinylation, upregulation of protein monoubiquitylation, activation of protein monoubiquitination, activation of protein monoubiquitinylation, activation of protein monoubiquitylation Definition: Any process that activates or increases the frequency, rate or extent of protein monoubiquitination.